{
  "term_id": "GO:0006886",
  "gene_name": "Vacuolar protein sorting-associated protein 45",
  "gene": "UniProtKB:Q9NRW7",
  "term_label": "intracellular protein transport",
  "gene_symbol": "VPS45"
}